{
  "gene": "UniProtKB:P10176",
  "gene_name": "Cytochrome c oxidase subunit 8A, mitochondrial",
  "term_label": "Unknown biological process",
  "gene_symbol": "COX8A",
  "term_id": "UNKNOWN:0002"
}